regulation of transcription initiation by RNA polymerase II [GO:0060260] (BP) Also known as: regulation of transcription initiation from RNA polymerase II promoter Sources: GOC:dph, GOC:tb, GOC:txnOH Subtypes: GO:0001178, GO:0045898, GO:0060261, GO:0060633 Relationships: is a type of regulation of transcription by RNA polymerase II [GO:0006357]; is a type of regulation of DNA-templated transcription initiation [GO:2000142]; regulates transcription initiation at RNA polymerase II promoter [GO:0006367] Definition: Any process that modulates the rate, frequency or extent of a process involved in starting transcription from an RNA polymerase II promoter.